polar nucleus [GO:0043078] (cellular component) Relationships: is a type of megasporocyte nucleus [GO:0043076] Sources: ISBN:0618254153 Definition: Either of two nuclei located centrally in a flowering plant embryo sac that eventually fuse to form the endosperm nucleus.